{
  "gene_name": "Olfactory receptor 1D4",
  "term_label": "plasma membrane",
  "gene_symbol": "OR1D4",
  "gene": "UniProtKB:P47884",
  "term_id": "GO:0005886"
}